{
  "term_label": "keratan sulfate proteoglycan biosynthetic process",
  "gene_name": "Carbohydrate sulfotransferase 6",
  "gene_symbol": "CHST6",
  "gene": "UniProtKB:Q9GZX3",
  "term_id": "GO:0018146"
}